{
  "gene_name": "A-kinase anchor protein 5",
  "gene_symbol": "AKAP5",
  "term_id": "GO:0060076",
  "term_label": "excitatory synapse",
  "gene": "UniProtKB:P24588"
}